{
  "gene": "UniProtKB:O43776",
  "term_id": "GO:0006421",
  "gene_symbol": "NARS1",
  "gene_name": "Asparagine--tRNA ligase, cytoplasmic",
  "term_label": "asparaginyl-tRNA aminoacylation"
}